{
  "gene_name": "Microfibrillar-associated protein 3-like",
  "term_id": "UNKNOWN:0002",
  "gene_symbol": "MFAP3L",
  "term_label": "Unknown biological process",
  "gene": "UniProtKB:O75121"
}